quorum sensing [GO:0009372] (biological process) References: PMID:10607620, PMID:15716452, PMID:16497924, PMID:16630813, PMID:8288518 Sources: GOC:krc, GOC:mlg Subtypes: host interaction involved in quorum sensing [GO:0120218] Also known as: quorum sensing system, cell-cell signaling involved in quorum sensing, detection of cell density by secreted molecule Definition: The cell-cell signaling process in which single-celled organisms carry out coordinated responses by monitoring their own population density, and often also that of other microbes, by producing small, diffusible, signal molecules, detecting the concentration of these molecules, and triggering a signal transduction pathway when a certain threshold is reached. Quorum sensing can occur amongst microbial communities in the environment or within host organisms. Relationships: is a type of cell-cell signaling [GO:0007267]; is a type of detection of cell density [GO:0060245]